{
  "gene_name": "Zinc finger protein 581",
  "term_label": "Unknown cellular component",
  "gene_symbol": "ZNF581",
  "term_id": "UNKNOWN:0003",
  "gene": "UniProtKB:Q9P0T4"
}